{
  "term_id": "GO:0050829",
  "term_label": "defense response to Gram-negative bacterium",
  "gene_name": "Toll-like receptor 4",
  "gene": "UniProtKB:O00206",
  "gene_symbol": "TLR4"
}